type 4 proteinase activated receptor binding [GO:0031875] (molecular function) Sources: GOC:mah, GOC:nln Definition: Binding to a type 4 proteinase activated receptor. Relationships: is a type of proteinase activated receptor binding [GO:0031871] Also known as: type 4 proteinase activated receptor ligand